{
  "gene_symbol": "ZKSCAN8",
  "term_id": "UNKNOWN:0003",
  "gene": "UniProtKB:Q15776",
  "term_label": "Unknown cellular component",
  "gene_name": "Zinc finger protein with KRAB and SCAN domains 8"
}